{
  "term_id": "GO:0005730",
  "gene_symbol": "RBM34",
  "gene_name": "RNA-binding protein 34",
  "term_label": "nucleolus",
  "gene": "UniProtKB:P42696"
}